neuromuscular junction of skeletal muscle fiber [GO:0098522] (cellular component) Definition: A neuromuscular junction in which the target muscle cell is a skeletal muscle fiber. Sources: GOC:dos Note: In vertebrates, the term 'neuromuscular junction' is limited to synapses targeting skeletal muscle fibers - all of which are cholinergic and excitatory. Both inhibitory and excitatory neuromuscular junctions exist in invertebrates, utilizing a range of neurotransmitters including glutamate, GABA and 5-HT. Relationships: is_a GO:0098520; is a type of GO:0098523; is_a GO:0098981